{
  "gene": "UniProtKB:O95049",
  "gene_name": "Tight junction protein ZO-3",
  "gene_symbol": "TJP3",
  "term_label": "cell-cell adhesion",
  "term_id": "GO:0098609"
}